negative regulation of chromosome segregation [GO:0051985] (biological process) Definition: Any process that stops, prevents, or reduces the frequency, rate or extent of chromosome segregation, the process in which genetic material, in the form of chromosomes, is organized and then physically separated and apportioned to two or more sets. Also known as: down regulation of chromosome segregation, down-regulation of chromosome segregation, downregulation of chromosome segregation, inhibition of chromosome segregation Relationships: is a type of negative regulation of cell cycle process [GO:0010948]; is a type of regulation of chromosome segregation [GO:0051983]; negatively regulates chromosome segregation [GO:0007059] Sources: GOC:ai Subtypes: negative regulation of sister chromatid segregation [GO:0033046], negative regulation of attachment of spindle microtubules to kinetochore [GO:0051986], GO:1905819